ocellus development [GO:0008056] (biological process) Definition: The process whose specific outcome is the progression of the ocellus over time, from its formation to the mature structure. The ocellus is a simple visual organ of insects. Sources: http://fly.ebi.ac.uk/.bin/cvreport2?id=FBcv0004540 Relationships: is a type of sensory organ development [GO:0007423]; is part of eye-antennal disc development [GO:0035214]